{
  "term_id": "GO:0050727",
  "gene_symbol": "SBNO2",
  "gene_name": "Protein strawberry notch homolog 2",
  "term_label": "regulation of inflammatory response",
  "gene": "UniProtKB:Q9Y2G9"
}